{
  "term_label": "regulation of cellular localization",
  "gene": "UniProtKB:Q9BYG5",
  "gene_symbol": "PARD6B",
  "gene_name": "Partitioning defective 6 homolog beta",
  "term_id": "GO:0060341"
}